{
  "term_id": "GO:0047493",
  "gene_symbol": "SAMD8",
  "term_label": "ceramide cholinephosphotransferase activity",
  "gene": "UniProtKB:Q96LT4",
  "gene_name": "Sphingomyelin synthase-related protein 1"
}